{
  "gene": "UniProtKB:P81277",
  "term_label": "prolactin-releasing peptide receptor binding",
  "gene_name": "Prolactin-releasing peptide",
  "gene_symbol": "PRLH",
  "term_id": "GO:0031861"
}